{
  "gene": "UniProtKB:Q9BQS6",
  "gene_name": "Heat shock protein beta-9",
  "gene_symbol": "HSPB9",
  "term_id": "UNKNOWN:0001",
  "term_label": "Unknown molecular function"
}